{
  "term_id": "GO:0014069",
  "gene_symbol": "NEGR1",
  "gene_name": "Neuronal growth regulator 1",
  "gene": "UniProtKB:Q7Z3B1",
  "term_label": "postsynaptic density"
}